regulation of systemic arterial blood pressure by carotid sinus baroreceptor feedback [GO:0001978] (biological process) Definition: The process that modulates blood pressure by sensing the amount of stretch occurring in large arteries and responding to the input via central nervous system control. Sources: GOC:dph, GOC:tb, ISBN:0721643949 Also known as: carotid sinus baroreceptor feedback regulation of systemic arterial blood pressure, baroreceptor feedback control of blood pressure, baroreceptor pressure buffer system Relationships: is a type of nervous system process involved in regulation of systemic arterial blood pressure [GO:0001976]; is part of regulation of systemic arterial blood pressure by baroreceptor feedback [GO:0003025] Subtypes: GO:0001982, baroreceptor response to increased systemic arterial blood pressure [GO:0001983]